{
  "term_id": "UNKNOWN:0001",
  "term_label": "Unknown molecular function",
  "gene_name": "Putative protein RFPL3S",
  "gene_symbol": "RFPL3S",
  "gene": "UniProtKB:P0C7P2"
}